axonemal microtubule [GO:0005879] (cellular component) Definition: A microtubule in the axoneme of a eukaryotic cilium or flagellum; an axoneme contains nine modified doublet microtubules, which may or may not surround a pair of single microtubules. Sources: GOC:cilia, ISBN:0815316194 Relationships: is a type of cytoplasmic microtubule [GO:0005881]; is part of axoneme [GO:0005930] Subtypes: GO:0097649, B axonemal microtubule [GO:0097650], GO:1990719, C2 axonemal microtubule [GO:1990720]